axon microtubule bundle [GO:1901589] (cellular component) Also known as: axon microtubule fascicle, microtubule bundle of axon, microtubule fascicle of axon Relationships: is a type of GO:0097427; BFO_0000050 axon [GO:0030424] Sources: GOC:TermGenie, NIF_Subcellular:sao707332678 Definition: An arrangement of closely apposed microtubules running parallel to each other in the axon hillock and initial segment.